{
  "gene_name": "Netrin-4",
  "gene": "UniProtKB:Q9HB63",
  "gene_symbol": "NTN4",
  "term_id": "GO:0043256",
  "term_label": "laminin complex"
}